negative regulation of fusion of sperm to egg plasma membrane [GO:0043013] (biological process) Definition: Any process that stops or prevents the binding and fusion of a sperm to the oocyte plasma membrane. References: PMID:34459848 Sources: GOC:jl Also known as: down regulation of fusion of sperm to egg plasma membrane, down-regulation of fusion of sperm to egg plasma membrane, downregulation of fusion of sperm to egg plasma membrane, inhibition of fusion of sperm to egg plasma membrane, inhibition of sperm-oocyte fusion, negative regulation of sperm-oocyte fusion Relationships: is a type of regulation of fusion of sperm to egg plasma membrane [GO:0043012]; is a type of negative regulation of cellular component organization [GO:0051129]; is a type of negative regulation of multicellular organismal process [GO:0051241]; is a type of negative regulation of reproductive process [GO:2000242]; negatively regulates fusion of sperm to egg plasma membrane involved in single fertilization [GO:0007342]